{
  "term_label": "DNA double-strand break processing",
  "term_id": "GO:0000729",
  "gene_symbol": "SMARCAD1",
  "gene_name": "SWI_SNF-related matrix-associated actin-dependent regulator of chromatin subfamily A containing DEAD_H box 1",
  "gene": "UniProtKB:Q9H4L7"
}